{
  "gene_symbol": "DMC1",
  "gene": "UniProtKB:Q14565",
  "term_label": "double-stranded DNA binding",
  "term_id": "GO:0003690",
  "gene_name": "Meiotic recombination protein DMC1_LIM15 homolog"
}